{
  "gene_symbol": "ACTBL2",
  "term_label": "NuA4 histone acetyltransferase complex",
  "term_id": "GO:0035267",
  "gene": "UniProtKB:Q562R1",
  "gene_name": "Beta-actin-like protein 2"
}